slow, calcium ion-dependent exocytosis of neurotransmitter [GO:0098747] (biological process) Definition: The slow, second phase of calcium ion-induced neurotransmitter release, via exocytosis, into the synaptic cleft. This depends on high affinity calcium sensors and decays slowly, typically with a decay constant of over 100ms. The underlying molecular mechanisms of this process are distinct from those of the earlier, fast phase of release. References: PMID:7809151, PMID:7954835 Sources: GOC:dos, GOC:pad, GOC:parl Relationships: is_a calcium ion-regulated exocytosis of neurotransmitter [GO:0048791]